{
  "term_label": "protein-cysteine S-palmitoyltransferase activity",
  "gene_name": "Palmitoyltransferase ZDHHC22",
  "gene_symbol": "ZDHHC22",
  "term_id": "GO:0019706",
  "gene": "UniProtKB:Q8N966"
}